Rab geranylgeranyltransferase activity [GO:0004663] (molecular function) Definition: Catalysis of the reaction: 2 geranylgeranyl diphosphate + protein-cysteine = 2 S-geranylgeranyl-protein + 2 diphosphate. This reaction is the formation of two thioether linkages between the C-1 atom of the geranylgeranyl groups and two cysteine residues within the terminal sequence motifs XXCC, XCXC or CCXX. Known substrates include Ras-related GTPases of a single family and the Rab family. References: PMID:8621375 Sources: EC:2.5.1.60, GOC:mah Also known as: GGTase-II activity, GGTaseII activity, Rab-protein geranylgeranyltransferase activity, RabGGTase activity, geranylgeranyl-diphosphate,geranylgeranyl-diphosphate:protein-cysteine geranyltransferase activity, protein geranylgeranyltransferase type II activity, type II protein geranyl-geranyltransferase activity Relationships: is a type of protein geranylgeranyltransferase activity [GO:0004661]